syn-isopimara-7,15-diene synthase activity [GO:0106243] (molecular function) References: PMID:29315936 Sources: GOC:emb, RHEA:62188 Definition: Catalysis of the reaction: 9alpha-copalyl diphosphate = diphosphate + syn-isopimara-7,15-diene. Relationships: is_a carbon-oxygen lyase activity, acting on phosphates [GO:0016838]